{
  "gene_symbol": "ALG10B",
  "term_label": "endoplasmic reticulum",
  "gene_name": "Putative Dol-P-Glc:Glc(2)Man(9)GlcNAc(2)-PP-Dol alpha-1,2-glucosyltransferase",
  "term_id": "GO:0005783",
  "gene": "UniProtKB:Q5I7T1"
}